{
  "gene_name": "Leucine-rich repeat neuronal protein 2",
  "term_id": "UNKNOWN:0002",
  "gene_symbol": "LRRN2",
  "term_label": "Unknown biological process",
  "gene": "UniProtKB:O75325"
}